plastid DNA metabolic process [GO:0033258] (biological process) Definition: The chemical reactions and pathways involving plastid DNA. Subtypes: plastid DNA replication [GO:0033259] Relationships: is a type of DNA metabolic process [GO:0006259]; is part of plastid organization [GO:0009657] Sources: GOC:mah Also known as: plastid DNA metabolism